{
  "term_label": "Unknown cellular component",
  "gene": "UniProtKB:Q9UHX1",
  "gene_symbol": "PUF60",
  "gene_name": "Poly(U)-binding-splicing factor PUF60",
  "term_id": "UNKNOWN:0003"
}